{
  "gene_name": "5-hydroxytryptamine receptor 2C",
  "term_id": "GO:0007187",
  "term_label": "G protein-coupled receptor signaling pathway, coupled to cyclic nucleotide second messenger",
  "gene_symbol": "HTR2C",
  "gene": "UniProtKB:P28335"
}